{
  "gene_name": "Membrane-associated guanylate kinase, WW and PDZ domain-containing protein 3",
  "gene": "UniProtKB:Q5TCQ9",
  "term_label": "cytoplasm",
  "gene_symbol": "MAGI3",
  "term_id": "GO:0005737"
}